{
  "term_id": "GO:0004725",
  "gene_name": "Dual specificity protein phosphatase CDC14C",
  "term_label": "protein tyrosine phosphatase activity",
  "gene_symbol": "CDC14C",
  "gene": "UniProtKB:A4D256"
}